{
  "term_label": "Unknown molecular function",
  "gene": "UniProtKB:Q5T2L2",
  "gene_symbol": "AKR1C8",
  "term_id": "UNKNOWN:0001",
  "gene_name": "Putative aldo-keto reductase family 1 member C8"
}